{
  "term_id": "GO:0007166",
  "gene_name": "T cell receptor beta variable 7-4",
  "gene": "UniProtKB:A0A1B0GX95",
  "term_label": "cell surface receptor signaling pathway",
  "gene_symbol": "TRBV7-4"
}